{
  "gene_name": "Tyrosine-protein phosphatase non-receptor type 12",
  "gene": "UniProtKB:Q05209",
  "term_id": "GO:0042058",
  "term_label": "regulation of epidermal growth factor receptor signaling pathway",
  "gene_symbol": "PTPN12"
}